{
  "gene_symbol": "SLC30A5",
  "term_id": "GO:0031410",
  "gene": "UniProtKB:Q8TAD4",
  "gene_name": "Proton-coupled zinc antiporter SLC30A5",
  "term_label": "cytoplasmic vesicle"
}